transmembrane receptor protein tyrosine kinase adaptor activity [GO:0005068] (molecular function) Relationships: is a type of signaling receptor complex adaptor activity [GO:0030159]; is a type of receptor tyrosine kinase binding [GO:0030971]; is part of cell surface receptor protein tyrosine kinase signaling pathway [GO:0007169] References: PMID:10502414, PMID:20565848 Sources: GOC:mtg_MIT_16mar07 Definition: The binding activity of a molecule that brings together a transmembrane receptor protein tyrosine kinase and one or more other molecules, permitting them to function in a coordinated way. Also known as: transmembrane receptor protein tyrosine kinase adaptor protein activity, transmembrane receptor protein tyrosine kinase docking protein activity